{
  "gene_symbol": "TBCC",
  "term_id": "GO:0005737",
  "gene": "UniProtKB:Q15814",
  "gene_name": "Tubulin-specific chaperone C",
  "term_label": "cytoplasm"
}